3-ketopimelyl-CoA thiolase activity [GO:0018713] (molecular function) Relationships: is a type of acyltransferase activity, transferring groups other than amino-acyl groups [GO:0016747] Definition: Catalysis of the reaction: 3-ketopimeloyl-CoA + CoA = glutaryl-CoA + acetyl-CoA. Sources: UM-BBD_reactionID:r0197